{
  "term_label": "regulation of calcium ion-dependent exocytosis",
  "gene": "UniProtKB:Q8IV01",
  "term_id": "GO:0017158",
  "gene_symbol": "SYT12",
  "gene_name": "Synaptotagmin-12"
}